regulation of CD4-positive, CD25-positive, alpha-beta regulatory T cell differentiation involved in immune response [GO:0032832] (biological process) Relationships: is a type of regulation of immune effector process [GO:0002697]; is a type of GO:0032829; is a type of regulation of immune response [GO:0050776]; regulates CD4-positive, CD25-positive, alpha-beta regulatory T cell differentiation involved in immune response [GO:0002298] Also known as: regulation of CD4-positive, CD25-positive, alpha-beta regulatory T cell development involved in immune response, regulation of CD4-positive, CD25-positive, alpha-beta regulatory T cell differentiation during immune response, regulation of CD4-positive, CD25-positive, alpha-beta regulatory T lymphocyte differentiation during immune response, regulation of CD4-positive, CD25-positive, alpha-beta regulatory T-cell differentiation during immune response, regulation of CD4-positive, CD25-positive, alpha-beta regulatory T-lymphocyte differentiation during immune response Definition: Any process that modulates the frequency, rate or extent of differentiation of CD4-positive, CD25-positive, alpha-beta regulatory T cells as part of an immune response. Subtypes: negative regulation of CD4-positive, CD25-positive, alpha-beta regulatory T cell differentiation involved in immune response [GO:0032833], positive regulation of CD4-positive, CD25-positive, alpha-beta regulatory T cell differentiation involved in immune response [GO:0032834] Note: Note that immunologists typically use the word 'development' to refer to cells of B or T cell lineages undergoing the process that GO describes as 'cell differentiation'. Sources: GOC:mah